{
  "term_label": "positive regulation of innate immune response",
  "gene": "UniProtKB:O15162",
  "gene_symbol": "PLSCR1",
  "term_id": "GO:0045089",
  "gene_name": "Phospholipid scramblase 1"
}